5S rDNA binding [GO:0080084] (molecular function) References: PMID:12711688 Relationships: is a type of rDNA binding [GO:0000182] Subtypes: RNA polymerase III type 1 promoter sequence-specific DNA binding [GO:0001002] Definition: Binding to a 5S rDNA sequence, encoding ribosomal 5S rRNA, which is individually transcribed by RNA polymerase III, rather than by RNA polymerase I, in species where it exists.